{
  "term_label": "Unknown molecular function",
  "gene": "UniProtKB:Q9BYZ8",
  "gene_name": "Regenerating islet-derived protein 4",
  "gene_symbol": "REG4",
  "term_id": "UNKNOWN:0001"
}